{
  "term_label": "Unknown cellular component",
  "gene_name": "Early activation antigen CD69",
  "gene": "UniProtKB:Q07108",
  "term_id": "UNKNOWN:0003",
  "gene_symbol": "CD69"
}